{
  "gene_symbol": "ENTPD1",
  "gene_name": "Ectonucleoside triphosphate diphosphohydrolase 1",
  "term_id": "GO:0045134",
  "term_label": "UDP phosphatase activity",
  "gene": "UniProtKB:P49961"
}